{
  "gene_name": "Dachshund homolog 1",
  "term_label": "nucleus",
  "gene": "UniProtKB:Q9UI36",
  "term_id": "GO:0005634",
  "gene_symbol": "DACH1"
}